{
  "term_id": "GO:0034381",
  "gene": "UniProtKB:P21757",
  "term_label": "plasma lipoprotein particle clearance",
  "gene_name": "Macrophage scavenger receptor types I and II",
  "gene_symbol": "MSR1"
}